aluminum cation transport [GO:0015690] (biological process) Also known as: aluminium ion transport, aluminium transport, aluminum transport, aluminum ion transport Definition: The directed movement of aluminum (Al) ions into, out of or within a cell, or between cells, by means of some agent such as a transporter or pore. Relationships: is a type of GO:0030001 Sources: GOC:ai